{
  "term_label": "COP9 signalosome",
  "gene": "UniProtKB:P62993",
  "term_id": "GO:0008180",
  "gene_name": "Growth factor receptor-bound protein 2",
  "gene_symbol": "GRB2"
}